tRNA(Ile)-lysidine synthase activity [GO:0032267] (molecular function) Definition: Catalysis of the reaction: ATP + cytidine(34) in tRNA(Ile2) + L-lysine = AMP + diphosphate + H+ + lysidine(34) in tRNA(Ile2). This modification converts both the codon specificity of tRNA(Ile) from AUG to AUA and its amino acid specificity from methionine to isoleucine. Also known as: tRNA(Ile)-2-lysyl-cytidine synthase activity, tRNA(Ile)-lysidine synthetase activity References: PMID:14527414 Sources: RHEA:43744 Relationships: is a type of GO:0016879; is a type of GO:0140101